mesonephric mesenchymal cell differentiation [GO:0061223] (biological process) Sources: GOC:mtg_kidney_jan10 Definition: The process in which relatively unspecialized cells acquire specialized structural and/or functional features that characterize the mesenchymal cells of the mesonephros as it progresses from its formation to the mature state. Relationships: is a type of cell differentiation involved in mesonephros development [GO:0061208]; is a type of GO:0072161; is part of GO:0061219